signal transduction involved in positive regulation of conjugation with cellular fusion [GO:0032005] (biological process) Definition: The series of molecular signals that bring about the relay, amplification or dampening of a signal generated in response to a cue, such as starvation or pheromone exposure, in organisms that undergo conjugation with cellular fusion. Sources: GOC:mah Regulation: regulated by regulation of signal transduction involved in conjugation with cellular fusion [GO:0060238]; positively regulated by positive regulation of signal transduction involved in conjugation with cellular fusion [GO:0060239]; negatively regulated by GO:0060240 Subtypes: pheromone-dependent signal transduction involved in conjugation with cellular fusion [GO:0000750] Relationships: is a type of signal transduction [GO:0007165]; is a type of positive regulation of conjugation with cellular fusion [GO:0031139]